{
  "term_label": "regulation of ERK1 and ERK2 cascade",
  "term_id": "GO:0070372",
  "gene": "UniProtKB:Q8WUJ0",
  "gene_name": "Serine_threonine_tyrosine-interacting protein",
  "gene_symbol": "STYX"
}